{
  "gene_symbol": "FMR1",
  "term_id": "GO:0005634",
  "term_label": "nucleus",
  "gene": "UniProtKB:Q06787",
  "gene_name": "Fragile X messenger ribonucleoprotein 1"
}